{
  "gene": "UniProtKB:Q07157",
  "gene_name": "Tight junction protein ZO-1",
  "term_label": "cell-cell junction organization",
  "term_id": "GO:0045216",
  "gene_symbol": "TJP1"
}